{
  "term_label": "small-subunit processome",
  "gene_symbol": "UTP11",
  "gene": "UniProtKB:Q9Y3A2",
  "gene_name": "Probable U3 small nucleolar RNA-associated protein 11",
  "term_id": "GO:0032040"
}